{
  "gene": "UniProtKB:P47902",
  "term_label": "cell differentiation",
  "term_id": "GO:0030154",
  "gene_symbol": "CDX1",
  "gene_name": "Homeobox protein CDX-1"
}